transmembrane receptor histidine kinase activity [GO:0009784] (molecular function) Relationships: is a type of protein histidine kinase activity [GO:0004673]; is_a transmembrane receptor protein kinase activity [GO:0019199] Sources: GOC:lr, GOC:mah Subtypes: transmembrane histidine kinase cytokinin receptor activity [GO:0009885] Definition: Combining with a signal and transmitting the signal from one side of a membrane to the other to initiate a change in cell activity by catalysis of the reaction: ATP + a protein-L-histidine = ADP + a protein-L-histidine phosphate.